{
  "term_label": "Unknown molecular function",
  "gene": "UniProtKB:A0A0G2JQF1",
  "gene_name": "Uncharacterized protein",
  "term_id": "UNKNOWN:0001",
  "gene_symbol": "A0A0G2JQF1"
}